response to diosgenin [GO:1905092] (biological process) Relationships: is a type of response to sterol [GO:0036314]; is a type of response to alcohol [GO:0097305]; is a type of response to triterpenoid [GO:1905836] Subtypes: cellular response to diosgenin [GO:1905093] Definition: Any process that results in a change in state or activity of a cell or an organism (in terms of movement, secretion, enzyme production, gene expression, etc.) as a result of a diosgenin stimulus. References: PMID:25765596 Sources: GOC:BHF, GOC:BHF_miRNA, GOC:TermGenie, GOC:bc, GO_REF:0000071